{
  "gene_name": "Nicotinamide_nicotinic acid mononucleotide adenylyltransferase 2",
  "term_label": "NAD+ biosynthetic process via the salvage pathway",
  "term_id": "GO:0034355",
  "gene": "UniProtKB:Q9BZQ4",
  "gene_symbol": "NMNAT2"
}